{
  "term_id": "GO:0034389",
  "gene_name": "Lipid droplet-associated hydrolase",
  "term_label": "lipid droplet organization",
  "gene_symbol": "LDAH",
  "gene": "UniProtKB:Q9H6V9"
}